{
  "gene_name": "Large ribosomal subunit protein mL53",
  "gene_symbol": "MRPL53",
  "term_id": "UNKNOWN:0002",
  "term_label": "Unknown biological process",
  "gene": "UniProtKB:Q96EL3"
}